{
  "term_label": "Unknown molecular function",
  "gene_symbol": "ZNF318",
  "gene": "UniProtKB:Q5VUA4",
  "term_id": "UNKNOWN:0001",
  "gene_name": "Zinc finger protein 318"
}